2-hydroxy-but-3-enyl glucosinolate biosynthetic process [GO:0080035] (biological process) Also known as: 2-hydroxy-but-3-enyl glucosinolate anabolism, 2-hydroxy-but-3-enyl glucosinolate biosynthesis, 2-hydroxy-but-3-enyl glucosinolate formation, 2-hydroxy-but-3-enyl glucosinolate synthesis, progoitrin biosynthesis, progoitrin biosynthetic process, progoitrin synthesis Relationships: is a type of GO:0019761; is a type of secondary alcohol biosynthetic process [GO:1902653] References: PMID:11560911, PMID:18945935 Definition: The chemical reactions and pathways resulting in the formation of progoitrin, a 2-hydroxy-but-3-enyl glucosinolate. Glucosinolates are substituted thioglucosides found in rapeseed products and related cruciferae, and progoitrin has been implicated in causing goiters in mammals and bitter taste in cruciferous vegetables.